symbiont-mediated suppression of host antigen processing and presentation of peptide antigen via MHC class II [GO:0039505] (biological process) Also known as: inhibition of host MHC class II molecule presentation by virus, suppression by virus of host antigen processing and presentation of peptide antigen via MHC class II Relationships: is a type of symbiont-mediated suppression of host antigen processing and presentation [GO:0039588] Definition: A process by which a symbiont inhibits or disrupts the normal processing and presentation of a peptide antigen on its cell surface in association with an MHC class II protein complex. References: PMID:27832589 Sources: GOC:add, GOC:bf, VZ:820